substrate-dependent cerebral cortex tangential migration [GO:0021825] (biological process) Relationships: is a type of substrate-dependent cell migration [GO:0006929]; is a type of cerebral cortex tangential migration [GO:0021800] Sources: GOC:cls, GOC:dgh, GOC:dph, GOC:jid, GO_REF:0000021 Subtypes: cerebral cortex tangential migration using cell-cell interactions [GO:0021823], cerebral cortex tangential migration using cell-axon interactions [GO:0021824] Definition: The process where neuronal precursors migrate tangentially in the cerebral cortex, primarily guided through physical cell-cell interactions.